{
  "gene": "UniProtKB:Q96EK2",
  "term_id": "UNKNOWN:0002",
  "gene_name": "PHD finger protein 21B",
  "gene_symbol": "PHF21B",
  "term_label": "Unknown biological process"
}